{
  "term_id": "GO:0005737",
  "gene_name": "Tubulin alpha-3C chain",
  "term_label": "cytoplasm",
  "gene": "UniProtKB:P0DPH7",
  "gene_symbol": "TUBA3C"
}